{
  "term_id": "UNKNOWN:0003",
  "gene": "UniProtKB:Q17RQ9",
  "term_label": "Unknown cellular component",
  "gene_symbol": "NKPD1",
  "gene_name": "NTPase KAP family P-loop domain-containing protein 1"
}